{
  "gene_symbol": "GNAI1",
  "term_label": "cytoplasm",
  "gene": "UniProtKB:P63096",
  "gene_name": "Guanine nucleotide-binding protein G(i) subunit alpha-1",
  "term_id": "GO:0005737"
}